{
  "gene_name": "MICOS complex subunit MIC60",
  "term_id": "UNKNOWN:0001",
  "gene": "UniProtKB:Q16891",
  "term_label": "Unknown molecular function",
  "gene_symbol": "IMMT"
}